{
  "gene_name": "Melanin-concentrating hormone receptor 1",
  "term_id": "GO:0007218",
  "gene": "UniProtKB:Q99705",
  "gene_symbol": "MCHR1",
  "term_label": "neuropeptide signaling pathway"
}